{
  "term_id": "UNKNOWN:0001",
  "term_label": "Unknown molecular function",
  "gene_name": "Cip1-interacting zinc finger protein",
  "gene": "UniProtKB:Q9ULV3",
  "gene_symbol": "CIZ1"
}